{
  "term_label": "calcium channel activity",
  "gene": "UniProtKB:Q9NZM6",
  "gene_symbol": "PKD2L2",
  "gene_name": "Polycystin-2-like protein 2",
  "term_id": "GO:0005262"
}